fibronectin-dependent thymocyte migration [GO:0072681] (biological process) Also known as: fibronectin-dependent thymic lymphocyte migration, fibronectin-dependent immature T cell migration, fibronectin-dependent immature T lymphocyte migration, fibronectin-dependent immature T-cell migration, fibronectin-dependent immature T-lymphocyte migration Relationships: is_a extracellular matrix-dependent thymocyte migration [GO:0072680] Definition: The movement of a thymocyte through distinct intrathymic niches (e.g. medulla, cortex), where it receives a unique set of developmental cues required for T-cell development, dependent on fibronectin in the extracellular matrix. References: PMID:20856819 Sources: CL:0000893, GOC:BHF, GOC:mah Regulation: regulated by regulation of fibronectin-dependent thymocyte migration [GO:2000413]; negatively regulated by negative regulation of fibronectin-dependent thymocyte migration [GO:2000414]; positively regulated by positive regulation of fibronectin-dependent thymocyte migration [GO:2000415]